{
  "gene_symbol": "BAZ1A",
  "gene": "UniProtKB:Q9NRL2",
  "term_id": "GO:0008623",
  "gene_name": "Bromodomain adjacent to zinc finger domain protein 1A",
  "term_label": "CHRAC"
}